{
  "term_label": "Unknown molecular function",
  "term_id": "UNKNOWN:0001",
  "gene_name": "Ankyrin repeat and SOCS box protein 3",
  "gene_symbol": "ASB3",
  "gene": "UniProtKB:Q9Y575"
}